cellular response to topologically incorrect protein [GO:0035967] (biological process) Definition: Any process that results in a change in state or activity of a cell (in terms of movement, secretion, enzyme production, gene expression, etc.) as a result of a protein that is not folded in its correct three-dimensional structure. Sources: GOC:bf Also known as: cellular response to misfolded or unfolded protein Relationships: is a type of cellular response to stress [GO:0033554]; is_a response to topologically incorrect protein [GO:0035966] Subtypes: cellular response to unfolded protein [GO:0034620], cellular response to misfolded protein [GO:0071218]